chloroplast proton-transporting ATP synthase complex assembly [GO:0033614] (biological process) Definition: The aggregation, arrangement and bonding together of a proton-transporting ATP synthase in the chloroplast thylakoid membrane. Relationships: is a type of proton-transporting ATP synthase complex assembly [GO:0043461]; is part of chloroplast organization [GO:0009658]; BFO_0000066 chloroplast [GO:0009507] Sources: GOC:mah